{
  "term_label": "nucleus",
  "term_id": "GO:0005634",
  "gene_name": "E3 ubiquitin-protein ligase MARCHF7",
  "gene": "UniProtKB:Q9H992",
  "gene_symbol": "MARCHF7"
}